{
  "gene_symbol": "ZSWIM8",
  "gene": "UniProtKB:A7E2V4",
  "gene_name": "Zinc finger SWIM domain-containing protein 8",
  "term_id": "GO:0031462",
  "term_label": "Cul2-RING ubiquitin ligase complex"
}